C-X3-C chemokine receptor activity [GO:0016495] (molecular function) Sources: GOC:dph, GOC:signaling Definition: Combining with a C-X3-C chemokine and transmitting the signal from one side of the membrane to the other to initiate a change in cell activity. A C-X3-C chemokine has three amino acids between the first two cysteines of the characteristic four-cysteine motif. Relationships: is a type of chemokine receptor activity [GO:0004950]; has part GO:0019960